{
  "term_id": "GO:0061697",
  "term_label": "protein-glutaryllysine deglutarylase activity",
  "gene": "UniProtKB:Q9NRC8",
  "gene_symbol": "SIRT7",
  "gene_name": "NAD-dependent protein deacetylase sirtuin-7"
}